{
  "term_id": "GO:0007229",
  "gene": "UniProtKB:Q13477",
  "gene_name": "Mucosal addressin cell adhesion molecule 1",
  "gene_symbol": "MADCAM1",
  "term_label": "integrin-mediated signaling pathway"
}